{
  "gene_name": "Remodeling and spacing factor 1",
  "term_id": "GO:0042393",
  "term_label": "histone binding",
  "gene_symbol": "RSF1",
  "gene": "UniProtKB:Q96T23"
}